{
  "gene_name": "Putative tyrosine-protein phosphatase auxilin",
  "gene": "UniProtKB:O75061",
  "gene_symbol": "DNAJC6",
  "term_label": "cytoplasm",
  "term_id": "GO:0005737"
}